negative regulation of macroautophagy [GO:0016242] (biological process) Relationships: is a type of negative regulation of autophagy [GO:0010507]; is a type of GO:0016241; negatively regulates GO:0016236 Definition: Any process that stops, prevents, or reduces the frequency, rate or extent of macroautophagy. Subtypes: GO:1901097, GO:1901525, GO:1902902, negative regulation of xenophagy [GO:1904416], negative regulation of lipophagy [GO:1904503], negative regulation of aggrephagy [GO:1905336] Also known as: down regulation of macroautophagy, down-regulation of macroautophagy, downregulation of macroautophagy, negative regulation of starvation-induced autophagy, inhibition of macroautophagy Sources: GOC:go_curators